purine phosphoribosyltransferase activity [GO:0106130] (MF) References: PMID:5123876 Relationships: is a type of GO:0016763 Definition: Catalysis of the reaction: RMP + diphosphate = R + 5-phospho-alpha-D-ribose 1-diphosphate. Subtypes: GO:0000310, adenine phosphoribosyltransferase activity [GO:0003999], hypoxanthine phosphoribosyltransferase activity [GO:0004422], GO:0052657